{
  "term_id": "GO:0033691",
  "term_label": "sialic acid binding",
  "gene": "UniProtKB:Q96PQ1",
  "gene_symbol": "SIGLEC12",
  "gene_name": "Sialic acid-binding Ig-like lectin 12"
}